{
  "gene_symbol": "LINC00310",
  "term_label": "Unknown biological process",
  "gene_name": "Putative uncharacterized protein encoded by LINC00310",
  "gene": "UniProtKB:P59036",
  "term_id": "UNKNOWN:0002"
}